{
  "gene_symbol": "ROCK1",
  "term_label": "cytoplasm",
  "gene_name": "Rho-associated protein kinase 1",
  "gene": "UniProtKB:Q13464",
  "term_id": "GO:0005737"
}